mitotic actomyosin contractile ring assembly actin filament organization [GO:1903479] (biological process) Definition: Any actin filament organization that is involved in mitotic actomyosin contractile ring assembly. Relationships: is a type of GO:1903047; is a type of actomyosin contractile ring assembly actin filament organization [GO:2000689]; is part of mitotic actomyosin contractile ring assembly [GO:1903475] Also known as: actin filament organisation involved in contractile ring assembly involved in mitotic cytokinesis, actin filament organisation involved in mitotic actomyosin contractile ring assembly, actin filament organization involved in mitotic actomyosin contractile ring assembly Subtypes: GO:1903477 Sources: GOC:TermGenie, GOC:mtg_cell_cycle, GO_REF:0000060